{
  "term_id": "GO:0008608",
  "gene_name": "BUB3-interacting and GLEBS motif-containing protein ZNF207",
  "term_label": "attachment of spindle microtubules to kinetochore",
  "gene": "UniProtKB:O43670",
  "gene_symbol": "ZNF207"
}